{
  "term_id": "UNKNOWN:0002",
  "term_label": "Unknown biological process",
  "gene": "UniProtKB:Q53RD9",
  "gene_name": "Fibulin-7",
  "gene_symbol": "FBLN7"
}